{
  "gene_name": "Far upstream element-binding protein 2",
  "term_id": "GO:0043488",
  "term_label": "regulation of mRNA stability",
  "gene_symbol": "KHSRP",
  "gene": "UniProtKB:Q92945"
}